{
  "gene": "UniProtKB:Q8N414",
  "term_label": "nucleus",
  "gene_name": "PiggyBac transposable element-derived protein 5",
  "term_id": "GO:0005634",
  "gene_symbol": "PGBD5"
}